positive regulation of eye pigmentation [GO:0048075] (biological process) Relationships: is a type of regulation of eye pigmentation [GO:0048073]; is a type of positive regulation of developmental pigmentation [GO:0048087]; positively regulates eye pigmentation [GO:0048069] Subtypes: positive regulation of compound eye pigmentation [GO:0048078] Definition: Any process that activates or increases the frequency, rate or extent of establishment of a pattern of pigment in the eye of an organism. Also known as: up regulation of eye pigmentation, up-regulation of eye pigmentation, upregulation of eye pigmentation, activation of eye pigmentation, stimulation of eye pigmentation Sources: GOC:jid